sperm midpiece [GO:0097225] (cellular component) Definition: The highly organized segment of the sperm flagellum which begins at the connecting piece and is characterized by the presence of 9 outer dense fibers (ODFs) that lie outside each of the 9 outer axonemal microtubule doublets and by a sheath of mitochondria that encloses the ODFs and the axoneme; the midpiece terminates about one-fourth of the way down the sperm flagellum at the annulus, which marks the beginning of the principal piece. Sources: GOC:cjm, MP:0009831 Relationships: is a type of cellular anatomical structure [GO:0110165]; is part of sperm flagellum [GO:0036126]